{
  "gene": "UniProtKB:Q9Y3C7",
  "term_label": "regulation of transcription by RNA polymerase II",
  "gene_symbol": "MED31",
  "term_id": "GO:0006357",
  "gene_name": "Mediator of RNA polymerase II transcription subunit 31"
}